{
  "gene_symbol": "POM121",
  "term_label": "structural constituent of nuclear pore",
  "term_id": "GO:0017056",
  "gene": "UniProtKB:Q96HA1",
  "gene_name": "Nuclear envelope pore membrane protein POM 121"
}